{
  "gene_symbol": "RAD9A",
  "gene_name": "Cell cycle checkpoint control protein RAD9A",
  "term_id": "GO:0006281",
  "gene": "UniProtKB:Q99638",
  "term_label": "DNA repair"
}